deoxyribonucleoside monophosphate biosynthetic process [GO:0009157] (biological process) Definition: The chemical reactions and pathways resulting in the formation of a deoxyribonucleoside monophosphate, a compound consisting of a nucleobase linked to a deoxyribose sugar esterified with phosphate on the sugar. Subtypes: purine deoxyribonucleoside monophosphate biosynthetic process [GO:0009171], pyrimidine deoxyribonucleoside monophosphate biosynthetic process [GO:0009177] Relationships: is a type of nucleoside monophosphate biosynthetic process [GO:0009124] Sources: GOC:go_curators, ISBN:0198506732 Also known as: deoxyribonucleoside monophosphate anabolism, deoxyribonucleoside monophosphate biosynthesis, deoxyribonucleoside monophosphate formation, deoxyribonucleoside monophosphate synthesis